negative regulation of ferroptosis [GO:0110076] (biological process) Relationships: is a type of negative regulation of programmed cell death [GO:0043069]; is a type of regulation of ferroptosis [GO:0110075]; negatively regulates ferroptosis [GO:0097707] Definition: Any process that stops, prevents, or reduces the frequency, rate or extent of ferroptosis. References: PMID:24439385, PMID:25402683, PMID:29290465 Sources: GOC:sp